{
  "term_id": "GO:0001227",
  "term_label": "DNA-binding transcription repressor activity, RNA polymerase II-specific",
  "gene_symbol": "ZGPAT",
  "gene_name": "Zinc finger CCCH-type with G patch domain-containing protein",
  "gene": "UniProtKB:Q8N5A5"
}